{
  "gene_symbol": "PITX3",
  "gene": "UniProtKB:O75364",
  "term_id": "GO:0005634",
  "gene_name": "Pituitary homeobox 3",
  "term_label": "nucleus"
}